{
  "gene_symbol": "TFPI2",
  "term_label": "serine-type endopeptidase inhibitor activity",
  "gene": "UniProtKB:P48307",
  "gene_name": "Tissue factor pathway inhibitor 2",
  "term_id": "GO:0004867"
}